{
  "gene_name": "Renalase",
  "gene": "UniProtKB:Q5VYX0",
  "term_id": "GO:0016651",
  "gene_symbol": "RNLS",
  "term_label": "oxidoreductase activity, acting on NAD(P)H"
}